{
  "gene": "UniProtKB:Q14118",
  "gene_name": "Dystroglycan 1",
  "term_label": "basement membrane",
  "gene_symbol": "DAG1",
  "term_id": "GO:0005604"
}